effector-mediated activation of plant hypersensitive response by symbiont [GO:0080185] (biological process) Relationships: is a type of GO:0034055; is a type of symbiont-mediated perturbation of host resistance gene-dependent defense response [GO:0052158] Definition: A symbiont process in which a molecule secreted by the symbiont activates a resistance gene-dependent defense response signaling pathway in the plant host, in order to activate a hypersensitive response to induce necrosis. In the plant, this process involves the direct or indirect recognition of the symbiont effector protein for example through plant resistance receptor or R proteins (or R genes). References: PMID:16497589, PMID:22241993, PMID:23411798, PMID:27641772 Also known as: activation by organism of defense response in host by specific elicitors, effector-triggered immunity, induction by organism of defense response in host by specific elicitors, induction by organism of pathogen-race/host plant cultivar-specific resistance in host, induction by organism of resistance gene-dependent defense response of other organism involved in symbiotic interaction, positive regulation by organism of defense response in host by specific elicitors, activation by organism of host gene-for-gene resistance, activation by organism of host resistance gene-dependent defense response, activation by symbiont of host resistance gene-dependent defense response, effector-mediated induction of plant hypersensitive response by symbiont, induction by organism of host gene-for-gene resistance, induction by symbiont of host resistance gene-dependent defense response, positive regulation by organism of host gene-for-gene resistance, positive regulation by symbiont of plant HR, positive regulation by symbiont of plant hypersensitive response, activation of HR, activation of hypersensitive response, ETI triggered of host innate immune response, ETI-triggered of host innate immune response, avirulence protein, effector-triggered induction of host innate immune response, effector-triggered induction of plant hypersensitive response by symbiont, effector-triggered necrosis, induction of effector-triggered immunity (ETI), necrotrophic effector, positive regulation by symbiont of host resistance gene-dependent defense response